{
  "term_label": "centrosome",
  "term_id": "GO:0005813",
  "gene": "UniProtKB:Q5BJF6",
  "gene_name": "Outer dense fiber protein 2",
  "gene_symbol": "ODF2"
}